regulation of neuron projection arborization [GO:0150011] (biological process) Relationships: is a type of GO:0022604; is a type of GO:0031344; regulates GO:0140058 Subtypes: positive regulation of neuron projection arborization [GO:0150012], negative regulation of neuron projection arborization [GO:0150013] Definition: Any process that modulates the frequency, rate or extent of the process in which the anatomical structures of a neuron projection are generated and organized into branches. Also known as: regulation of neurite arborization, regulation of neurite branching, regulation of neuron projection branching References: PMID:17114044 Sources: GOC:aruk, GOC:bc